{
  "gene_name": "Envoplakin-like protein",
  "term_label": "Unknown biological process",
  "gene": "UniProtKB:A8MZ36",
  "term_id": "UNKNOWN:0002",
  "gene_symbol": "EVPLL"
}